{
  "term_label": "spermatogenesis",
  "gene": "UniProtKB:Q96M20",
  "gene_name": "Cyclic nucleotide-binding domain-containing protein 2",
  "gene_symbol": "CNBD2",
  "term_id": "GO:0007283"
}